{
  "term_label": "ubiquitin-dependent protein catabolic process",
  "gene": "UniProtKB:Q9Y2X8",
  "gene_symbol": "UBE2D4",
  "gene_name": "Ubiquitin-conjugating enzyme E2 D4",
  "term_id": "GO:0006511"
}